{
  "term_id": "GO:0015459",
  "term_label": "potassium channel regulator activity",
  "gene_symbol": "KCNV2",
  "gene_name": "Potassium voltage-gated channel subfamily V member 2",
  "gene": "UniProtKB:Q8TDN2"
}